lactoferrin transport [GO:0033571] (biological process) Sources: GOC:mlg Definition: The directed movement of lactoferrin into, out of or within a cell, or between cells, by means of some agent such as a transporter or pore. Relationships: is a type of GO:0006826; is a type of protein transport [GO:0015031]